{
  "gene_name": "Ubiquitin-conjugating enzyme E2 E1",
  "gene_symbol": "UBE2E1",
  "gene": "UniProtKB:P51965",
  "term_id": "GO:0005634",
  "term_label": "nucleus"
}